{
  "gene": "UniProtKB:A3KMH1",
  "gene_name": "von Willebrand factor A domain-containing protein 8",
  "term_id": "GO:0005737",
  "term_label": "cytoplasm",
  "gene_symbol": "VWA8"
}